actomyosin contractile ring assembly [GO:0000915] (BP) Definition: The process of assembly of a ring composed of actin, myosin, and associated proteins that will function in cytokinesis. Sources: GOC:clt, GOC:dph, GOC:tb Also known as: contractile ring assembly, cytokinesis, actomyosin contractile ring assembly, constriction ring assembly, cytokinesis, actomyosin contractile ring formation, cytokinesis, actomyosin ring biosynthesis, cytokinesis, actomyosin ring formation, cytokinesis, contractile ring assembly, myosin filament organisation involved in cytokinetic actomyosin contractile ring assembly, myosin filament organization involved in cytokinetic actomyosin contractile ring assembly, myosin filament organization of constriction ring assembly, myosin filament organization of contractile ring assembly Relationships: is a type of assembly of actomyosin apparatus involved in cytokinesis [GO:0000912]; is a type of actomyosin contractile ring organization [GO:0044837] Subtypes: GO:1903475 Regulation: regulated by GO:2000431; negatively regulated by negative regulation of cytokinesis, actomyosin contractile ring assembly [GO:2000432]; positively regulated by positive regulation of cytokinesis, actomyosin contractile ring assembly [GO:2000433]